{
  "term_label": "plasma membrane",
  "gene_symbol": "MMP16",
  "gene": "UniProtKB:P51512",
  "term_id": "GO:0005886",
  "gene_name": "Matrix metalloproteinase-16"
}